{
  "term_id": "GO:0005829",
  "gene": "UniProtKB:P36871",
  "gene_symbol": "PGM1",
  "gene_name": "Phosphoglucomutase-1",
  "term_label": "cytosol"
}